aliphatic aldoxime dehydratase activity [GO:0034013] (MF) Sources: RHEA:11316 Relationships: is a type of nitrogen-oxygen lyase activity [GO:0141122] Also known as: aliphatic aldoxime hydro-lyase activity Definition: Catalysis of the reaction: an aliphatic aldoxime = an aliphatic nitrile + H2O.